D-amino acid transport [GO:0042940] (biological process) Definition: The directed movement of the D-enantiomer of an amino acid into, out of or within a cell, or between cells, by means of some agent such as a transporter or pore. Sources: GOC:jl, GOC:jsg, GOC:mah Relationships: is a type of amino acid transport [GO:0006865]; is a type of carboxylic acid transport [GO:0046942]; is a type of nitrogen compound transport [GO:0071705] Subtypes: D-alanine transmembrane transport [GO:0042941], D-serine transmembrane transport [GO:0042942], D-methionine transmembrane transport [GO:0048473], D-aspartate transmembrane transport [GO:0070777]